{
  "gene_symbol": "ETNK2",
  "gene": "UniProtKB:Q9NVF9",
  "term_label": "ethanolamine kinase activity",
  "term_id": "GO:0004305",
  "gene_name": "Ethanolamine kinase 2"
}